{
  "gene_symbol": "PLA2G4D",
  "term_label": "calcium-dependent phospholipase A2 activity",
  "gene": "UniProtKB:Q86XP0",
  "gene_name": "Cytosolic phospholipase A2 delta",
  "term_id": "GO:0047498"
}